{
  "term_label": "Unknown biological process",
  "gene": "UniProtKB:Q02223",
  "term_id": "UNKNOWN:0002",
  "gene_name": "Tumor necrosis factor receptor superfamily member 17",
  "gene_symbol": "TNFRSF17"
}